{
  "term_label": "N-acylphosphatidylethanolamine metabolic process",
  "term_id": "GO:0070292",
  "gene_name": "Phospholipase A and acyltransferase 1",
  "gene": "UniProtKB:Q9HDD0",
  "gene_symbol": "PLAAT1"
}